cyclin B2-CDK1 complex [GO:0097126] (cellular component) Relationships: is a type of GO:0000307 Definition: A protein complex consisting of cyclin B2 and cyclin-dependent kinase 1 (CDK1). Cyclins are characterized by periodicity in protein abundance throughout the cell cycle. Cyclin-dependent kinases represent a family of serine/threonine protein kinases that become active upon binding to a cyclin regulatory partner. References: PMID:15935619 Sources: GOC:so